{
  "gene_name": "Sodium_hydrogen exchanger 9",
  "term_id": "GO:0005886",
  "gene_symbol": "SLC9A9",
  "gene": "UniProtKB:Q8IVB4",
  "term_label": "plasma membrane"
}